positive regulation of translation in response to osmotic stress [GO:0032062] (biological process) Definition: Any process that activates or increases the frequency, rate or extent of translation as a result of a stimulus indicating an increase or decrease in the concentration of solutes outside the organism or cell. Also known as: up regulation of translation in response to osmotic stress, up-regulation of translation in response to osmotic stress, upregulation of translation in response to osmotic stress, activation of translation in response to osmotic stress, stimulation of translation in response to osmotic stress Sources: GOC:mah Relationships: is a type of positive regulation of translation in response to stress [GO:0032056]; is a type of regulation of translation in response to osmotic stress [GO:0043557] Subtypes: positive regulation of translational initiation in response to osmotic stress [GO:0032064]